{
  "gene_symbol": "DNAJC22",
  "term_id": "UNKNOWN:0002",
  "gene": "UniProtKB:Q8N4W6",
  "term_label": "Unknown biological process",
  "gene_name": "DnaJ homolog subfamily C member 22"
}